{
  "gene": "UniProtKB:Q9P2L0",
  "term_id": "GO:0030991",
  "term_label": "intraciliary transport particle A",
  "gene_symbol": "WDR35",
  "gene_name": "WD repeat-containing protein 35"
}